{
  "gene": "UniProtKB:P43235",
  "term_id": "GO:0004197",
  "gene_name": "Cathepsin K",
  "gene_symbol": "CTSK",
  "term_label": "cysteine-type endopeptidase activity"
}